regulation of calcium ion binding [GO:1901876] (biological process) Relationships: is_a GO:0051098; regulates calcium ion binding [GO:0005509] References: PMID:16432188 Sources: GOC:BHF, GOC:TermGenie, GOC:rl Definition: Any process that modulates the frequency, rate or extent of calcium ion binding. Also known as: regulation of calcium ion storage activity